{
  "gene_name": "Nuclear envelope pore membrane protein POM 121C",
  "term_label": "RNA export from nucleus",
  "term_id": "GO:0006405",
  "gene": "UniProtKB:A8CG34",
  "gene_symbol": "POM121C"
}